{
  "gene_name": "Long-chain fatty acid transport protein 6",
  "term_id": "GO:0005324",
  "gene_symbol": "SLC27A6",
  "term_label": "long-chain fatty acid transmembrane transporter activity",
  "gene": "UniProtKB:Q9Y2P4"
}